{
  "gene": "UniProtKB:A0A0U1RQG5",
  "term_id": "UNKNOWN:0002",
  "gene_name": "Cancer_testis antigen family 47 member C1",
  "gene_symbol": "CT47C1",
  "term_label": "Unknown biological process"
}